{
  "gene_name": "Coiled-coil domain-containing protein 28A",
  "gene": "UniProtKB:Q8IWP9",
  "gene_symbol": "CCDC28A",
  "term_id": "UNKNOWN:0002",
  "term_label": "Unknown biological process"
}